interleukin-22 receptor activity [GO:0042018] (MF) Relationships: is a type of cytokine receptor activity [GO:0004896]; is part of interleukin-22-mediated signaling pathway [GO:0140865]; has part interleukin-22 binding [GO:0042017] Sources: GOC:jl, GOC:signaling Also known as: IL-22 receptor activity, IL-22R Definition: Combining with interleukin-22 and transmitting the signal from one side of the membrane to the other to initiate a change in cell activity.